{
  "term_id": "GO:0005789",
  "gene": "UniProtKB:Q96BY9",
  "gene_name": "Store-operated calcium entry-associated regulatory factor",
  "term_label": "endoplasmic reticulum membrane",
  "gene_symbol": "SARAF"
}